{
  "gene_name": "MAP kinase-interacting serine_threonine-protein kinase 1",
  "term_id": "GO:0035556",
  "gene": "UniProtKB:Q9BUB5",
  "term_label": "intracellular signal transduction",
  "gene_symbol": "MKNK1"
}